positive regulation of neuron projection development [GO:0010976] (biological process) Definition: Any process that increases the rate, frequency or extent of neuron projection development. Neuron projection development is the process whose specific outcome is the progression of a neuron projection over time, from its formation to the mature structure. A neuron projection is any process extending from a neural cell, such as axons or dendrites (collectively called neurites). Sources: GOC:dph, GOC:tb Also known as: positive regulation of neurite biosynthesis, positive regulation of neurite development, positive regulation of neurite formation, positive regulation of neurite growth Relationships: is a type of regulation of neuron projection development [GO:0010975]; is a type of positive regulation of cell projection organization [GO:0031346]; positively regulates neuron projection development [GO:0031175] Subtypes: GO:0061003, positive regulation of neuron projection regeneration [GO:0070572], positive regulation of dendrite development [GO:1900006], positive regulation of axon guidance [GO:1902669]